{
  "term_label": "nucleus",
  "gene_symbol": "KIF23",
  "gene": "UniProtKB:Q02241",
  "gene_name": "Kinesin-like protein KIF23",
  "term_id": "GO:0005634"
}